{
  "term_id": "GO:0006457",
  "gene_name": "DnaJ homolog subfamily C member 25",
  "gene": "UniProtKB:Q9H1X3",
  "term_label": "protein folding",
  "gene_symbol": "DNAJC25"
}